{
  "gene_name": "Zinc finger protein 540",
  "gene": "UniProtKB:Q8NDQ6",
  "term_label": "DNA-binding transcription factor activity, RNA polymerase II-specific",
  "term_id": "GO:0000981",
  "gene_symbol": "ZNF540"
}